{
  "term_label": "DNA-binding transcription factor activity, RNA polymerase II-specific",
  "gene_symbol": "ZNF18",
  "gene_name": "Zinc finger protein 18",
  "gene": "UniProtKB:P17022",
  "term_id": "GO:0000981"
}